positive regulation of calcium-mediated signaling [GO:0050850] (biological process) Definition: Any process that activates or increases the frequency, rate or extent of calcium-mediated signaling. Also known as: positive regulation of calcium-mediated signalling, up regulation of calcium-mediated signaling, up-regulation of calcium-mediated signaling, upregulation of calcium-mediated signaling, activation of calcium-mediated signaling, stimulation of calcium-mediated signaling Sources: GOC:ai Relationships: is a type of GO:0050848; is a type of GO:1902533; positively regulates calcium-mediated signaling [GO:0019722] Subtypes: positive regulation of calcineurin-mediated signaling [GO:0106058], positive regulation of calcium-mediated signaling involved in cellular response to salt stress [GO:1901196], positive regulation of calcium-mediated signaling involved in cellular response to calcium ion [GO:1901197], positive regulation of CAMKK-AMPK signaling cascade [GO:1905291]